{
  "gene": "UniProtKB:P48730",
  "term_id": "GO:1905515",
  "term_label": "non-motile cilium assembly",
  "gene_symbol": "CSNK1D",
  "gene_name": "Casein kinase I isoform delta"
}